L-histidine transmembrane import into vacuole [GO:0090513] (biological process) Definition: The directed movement of L-histidine into the vacuole across the vacuolar membrane. Sources: GOC:al Relationships: is a type of basic amino acid transmembrane import into vacuole [GO:0034490]; is a type of GO:0089709; is a type of L-histidine transport [GO:1902024] Also known as: histidine transmembrane import into vacuole, vacuolar histidine import